{
  "term_id": "UNKNOWN:0002",
  "term_label": "Unknown biological process",
  "gene_name": "Epidermal growth factor-like protein 6",
  "gene": "UniProtKB:Q8IUX8",
  "gene_symbol": "EGFL6"
}